snoRNA 2,2,7-trimethylguanosine (TMG) capping [GO:0180031] (biological process) Subtypes: box C/D sno(s)RNA 5'-end processing [GO:0106410] Also known as: snoRNA 2,2,7-trimethylguanosine (TMG) cap formation, snoRNA capping References: PMID:15590684 Sources: GOC:vw Relationships: is a type of RNA capping [GO:0036260]; is a type of sno(s)RNA processing [GO:0043144] Definition: The sequence of enzymatic reactions by which a 2,2,7-trimethylguanosine cap structure is added to the 5' end of an snoRNA. The snoRNA capping includes the formation of 7-methyl-G caps found on all RNA polymerase II transcripts, followed by hypermethylation at the 2' position of the guanosine residue to convert a mono-methylated cap to a 2,2,7-trimethylguanosine cap structure. Note that the pol III transcribed snoRNAs are also TMG capped.